{
  "gene_symbol": "POF1B",
  "gene": "UniProtKB:Q8WVV4",
  "gene_name": "Protein POF1B",
  "term_id": "GO:0005912",
  "term_label": "adherens junction"
}